{
  "gene_symbol": "APBA1",
  "gene": "UniProtKB:Q02410",
  "term_label": "cytoplasm",
  "gene_name": "Amyloid-beta A4 precursor protein-binding family A member 1",
  "term_id": "GO:0005737"
}